{
  "term_id": "GO:0005634",
  "term_label": "nucleus",
  "gene": "UniProtKB:A8MUK1",
  "gene_name": "Ubiquitin carboxyl-terminal hydrolase 17-like protein 5",
  "gene_symbol": "USP17L5"
}